amino acid catabolic process via Ehrlich pathway [GO:0000955] (biological process) Subtypes: amino acid catabolic process to alcohol via Ehrlich pathway [GO:0000947], amino acid catabolic process to carboxylic acid via Ehrlich pathway [GO:0000948] Definition: The chemical reactions and pathways involving the catabolism of amino acids to produce alcohols or carboxylic acids containing one carbon less than the starting amino acid. In S. cerevisiae, this is known to occur for leucine, isoleucine, valine, methionine, phenylalanine, tyrosine, or tryptophan. Often referred to as the Ehrlich pathway, these reactions generally occur during fermentation to produce a variety of alcohols, often collectively referred to as fusel alcohols. Depending on the redox state of the cells, carboxylic acid derivatives, sometimes referred to as fusel acids, may be produced instead of alcohols. References: PMID:18281432 Sources: GOC:krc Relationships: is a type of amino acid catabolic process [GO:0009063]